hair follicle cell proliferation [GO:0071335] (BP) References: PMID:16086254 Sources: GOC:rph Relationships: is a type of cell population proliferation [GO:0008283] Definition: The multiplication or reproduction of hair follicle cells, resulting in the expansion of a cell population. Regulation: regulated by GO:0071336; negatively regulated by negative regulation of hair follicle cell proliferation [GO:0071337]; positively regulated by positive regulation of hair follicle cell proliferation [GO:0071338]